subtelomeric heterochromatin [GO:0140720] (cellular component) Relationships: is a type of heterochromatin [GO:0000792]; is part of chromosome, subtelomeric region [GO:0099115] Definition: Heterochromatin that is located adjacent to the telomere, and characterized by methylated H3 histone at lysine 9 (H3K9me2/H3K9me3). References: PMID:34576871